{
  "gene": "UniProtKB:Q8NBV8",
  "term_label": "plasma membrane",
  "gene_symbol": "SYT8",
  "term_id": "GO:0005886",
  "gene_name": "Synaptotagmin-8"
}